oligosaccharide 4-alpha-D-glucosyltransferase activity [GO:0033825] (molecular function) Sources: EC:2.4.1.161 Also known as: 1,4-alpha-D-glucan:1,4-alpha-D-glucan 4-alpha-D-glucosyltransferase activity, 1,4-alpha-glucan:1,4-alpha-glucan 4-alpha-glucosyltransferase activity, amylase III activity Definition: Catalysis of the transfer of the non-reducing terminal alpha-D-glucose residue from a 1,4-alpha-D-glucan to the 4-position of an alpha-D-glucan, thus bringing about the hydrolysis of oligosaccharides. Relationships: is a type of GO:0046527